{
  "gene_symbol": "AP4E1",
  "term_label": "cargo adaptor activity",
  "gene": "UniProtKB:Q9UPM8",
  "term_id": "GO:0140312",
  "gene_name": "AP-4 complex subunit epsilon-1"
}